response to testosterone [GO:0033574] (biological process) Subtypes: cellular response to testosterone stimulus [GO:0071394] Also known as: response to testosterone stimulus Relationships: is a type of GO:0033993; is a type of response to ketone [GO:1901654] Sources: GOC:sl Definition: Any process that results in a change in state or activity of a cell or an organism (in terms of movement, secretion, enzyme production, gene expression, etc.) as a result of a testosterone stimulus.